{
  "gene_name": "Complement C3",
  "gene": "UniProtKB:P01024",
  "gene_symbol": "C3",
  "term_id": "UNKNOWN:0001",
  "term_label": "Unknown molecular function"
}